membrane protein intracellular domain proteolysis [GO:0031293] (biological process) Relationships: is a type of GO:0033619 Subtypes: GO:0035333 Also known as: membrane protein solubilization Definition: The proteolytic cleavage of a transmembrane protein leading to the release of an intracellular domain. References: PMID:12808018